interleukin-23 receptor activity [GO:0042020] (molecular function) Also known as: IL-23 receptor activity, IL-23R Relationships: is a type of cytokine receptor activity [GO:0004896]; is part of interleukin-23-mediated signaling pathway [GO:0038155]; has part interleukin-23 binding [GO:0042019] Sources: GOC:jl, GOC:signaling Definition: Combining with interleukin-23 and transmitting the signal from one side of the membrane to the other to initiate a change in cell activity.